transitional two stage B cell differentiation [GO:0002334] (biological process) Sources: GOC:jal, ISBN:0781735149 Definition: The process in which immature B cells from the bone marrow acquire the specialized features of T2 stage B cells in the spleen. T2 stage B cells express CD23 but not CD21. Note: Note that immunologists typically use the word 'development' to refer to cells of B or T cell lineages undergoing the process that GO describes as 'cell differentiation'. Relationships: is a type of transitional stage B cell differentiation [GO:0002332] Also known as: T2 stage B cell differentiation, transitional two stage B lymphocyte differentiation, transitional two stage B-cell differentiation, transitional two stage B-lymphocyte differentiation, transitional two stage B cell development